{
  "gene_name": "ZW10 interactor",
  "term_label": "kinetochore",
  "gene": "UniProtKB:O95229",
  "term_id": "GO:0000776",
  "gene_symbol": "ZWINT"
}